{
  "gene": "UniProtKB:Q96KP1",
  "gene_name": "Exocyst complex component 2",
  "term_label": "exocytosis",
  "term_id": "GO:0006887",
  "gene_symbol": "EXOC2"
}